{
  "gene": "UniProtKB:A0A1W2PPE3",
  "term_label": "Unknown biological process",
  "gene_name": "Uncharacterized protein C1orf202",
  "term_id": "UNKNOWN:0002",
  "gene_symbol": "C1orf202"
}